{
  "gene_symbol": "GIMAP6",
  "gene": "UniProtKB:Q6P9H5",
  "gene_name": "GTPase IMAP family member 6",
  "term_id": "GO:0005829",
  "term_label": "cytosol"
}